{
  "term_label": "Unknown biological process",
  "gene": "UniProtKB:B6SEH9",
  "term_id": "UNKNOWN:0002",
  "gene_name": "Endogenous retrovirus group V member 2 Env polyprotein",
  "gene_symbol": "ERVV-2"
}